{
  "gene_name": "Epididymal-specific lipocalin-12",
  "term_label": "Unknown molecular function",
  "term_id": "UNKNOWN:0001",
  "gene_symbol": "LCN12",
  "gene": "UniProtKB:Q6JVE5"
}